{
  "term_label": "cell-cell adhesion mediated by cadherin",
  "gene": "UniProtKB:Q9Y6N8",
  "gene_name": "Cadherin-10",
  "term_id": "GO:0044331",
  "gene_symbol": "CDH10"
}